dopamine neurotransmitter receptor activity, coupled via Gi/Go [GO:0001591] (molecular function) Also known as: dopamine D2 receptor activity, dopamine D3 receptor activity, dopamine D4 receptor activity Relationships: is a type of dopamine neurotransmitter receptor activity [GO:0004952] Definition: Combining with the neurotransmitter dopamine and activating adenylate cyclase via coupling to Gi/Go to initiate a change in cell activity. Sources: GOC:mah, ISBN:0953351033, IUPHAR_RECEPTOR:2254, IUPHAR_RECEPTOR:2256, IUPHAR_RECEPTOR:2258